positive regulation of cytolysis [GO:0045919] (biological process) Also known as: up regulation of cytolysis, up-regulation of cytolysis, upregulation of cytolysis, activation of cytolysis, stimulation of cytolysis Sources: GOC:go_curators Relationships: is a type of regulation of cytolysis [GO:0042268]; is a type of positive regulation of cellular process [GO:0048522]; positively regulates cytolysis [GO:0019835] Definition: Any process that activates or increases the frequency, rate or extent of cytolysis.